{
  "gene_name": "Ubiquitin carboxyl-terminal hydrolase BAP1",
  "gene_symbol": "BAP1",
  "gene": "UniProtKB:Q92560",
  "term_label": "cysteine-type deubiquitinase activity",
  "term_id": "GO:0004843"
}